IPAF inflammasome complex [GO:0072557] (cellular component) Definition: An inflammasome complex that consists of three components, IPAF, NAIP and caspase-1, and includes among its functions the sensing of flagellin derived from Legionella pneumophila, Salmonella typhimurium, Pseudomonas aeruginosa and Shigella flexneri. References: PMID:20303873 Sources: GOC:BHF, GOC:add, GOC:vp Relationships: is a type of GO:0061702